calcium-dependent ATPase activity [GO:0030899] (molecular function) Relationships: is a type of ATP-dependent activity [GO:0140657] Regulation: negatively regulated by negative regulation of calcium-dependent ATPase activity [GO:1903611]; positively regulated by GO:1903612 Definition: Catalysis of the reaction: ATP + H2O = ADP + phosphate. This reaction requires the presence of calcium ion (Ca2+). Sources: GOC:mah